{
  "term_id": "GO:0005549",
  "gene_symbol": "OR5L1",
  "gene": "UniProtKB:Q8NGL2",
  "term_label": "odorant binding",
  "gene_name": "Olfactory receptor 5L1"
}